{
  "term_label": "dendrite",
  "term_id": "GO:0030425",
  "gene_symbol": "VSTM5",
  "gene_name": "V-set and transmembrane domain-containing protein 5",
  "gene": "UniProtKB:A8MXK1"
}